{
  "gene_symbol": "CHST12",
  "term_label": "sulfotransferase activity",
  "term_id": "GO:0008146",
  "gene": "UniProtKB:Q9NRB3",
  "gene_name": "Carbohydrate sulfotransferase 12"
}